negative regulation of membrane permeability [GO:1905709] (biological process) Definition: Any process that stops, prevents or reduces the frequency, rate or extent of the passage or uptake of molecules by a membrane. Relationships: is a type of GO:0090559 Subtypes: negative regulation of mitochondrial membrane permeability [GO:0035795], negative regulation of lysosomal membrane permeability [GO:0097215] References: PMID:27482894